regulation of ovarian follicle development [GO:2000354] (biological process) Relationships: is a type of regulation of developmental process [GO:0050793]; regulates GO:0001541 Subtypes: GO:2000355, GO:2000386 Definition: Any process that modulates the frequency, rate or extent of ovarian follicle development. Sources: GOC:obol Also known as: regulation of follicular phase